gut granule membrane [GO:0044841] (cellular component) Definition: The membrane of a gut granule, a lysosome-related organelle contained within the intestinal cells of the nematode C. elegans. References: PMID:22916203, PMID:24204312 Sources: GOC:kmv Relationships: is a type of cytoplasmic vesicle membrane [GO:0030659]; is part of gut granule [GO:0044840]